positive regulation of uredinium development [GO:0075281] (biological process) Sources: GOC:pamgo_curators Relationships: is a type of positive regulation of spore-bearing organ development [GO:0075261]; is a type of regulation of uredinium development [GO:0075280]; positively regulates uredinium development [GO:0075279] Definition: Any process that activates, maintains or increases the frequency, rate or extent of uredinium development, a process that leads to the formation of a reddish, pustule-like structure formed by a rust fungus and consisting of uredospores.